sequestering of TGFbeta in extracellular matrix [GO:0035583] (biological process) Definition: Confining TGFbeta to the extracellular matrix (ECM) such that it is separated from other components of the signaling pathway, including its cell surface receptor. TGFbeta is secreted as part of a latent complex that is targeted to the extracellular matrix through latent-TGFbeta-binding protein (LTBP)-mediated association with matrix proteins. References: PMID:12482908, PMID:20855508 Sources: GOC:BHF, GOC:bf, GOC:signaling Also known as: negative regulation of transforming growth factor beta receptor signaling pathway by extracellular matrix sequestering of TGFbeta, negative regulation of transforming growth factor beta receptor signalling pathway by extracellular matrix sequestering of TGFbeta, sequestering of TGFbeta LLC in extracellular matrix, sequestering of TGFbeta large latency complex in extracellular matrix Relationships: is a type of GO:0030512; is a type of sequestering of extracellular ligand from receptor [GO:0035581]; is a type of maintenance of protein location in extracellular region [GO:0071694]